{
  "gene": "UniProtKB:A0A0C4DH67",
  "gene_symbol": "IGKV1-8",
  "term_label": "immunoglobulin complex",
  "term_id": "GO:0019814",
  "gene_name": "Immunoglobulin kappa variable 1-8"
}